{
  "term_label": "nucleus",
  "gene_symbol": "RBM47",
  "term_id": "GO:0005634",
  "gene": "UniProtKB:A0AV96",
  "gene_name": "RNA-binding protein 47"
}